adenylate cyclase-inhibiting adrenergic receptor signaling pathway [GO:0071881] (biological process) Definition: An adenylate cyclase-inhibiting G protein-coupled receptor signaling pathway initiated by a ligand binding to an adrenergic receptor, and ending with the regulation of a downstream cellular process. Sources: GOC:BHF, GOC:mah, GOC:signaling Also known as: adrenergic receptor, adenylate cyclase inhibiting pathway, adrenergic receptor, adenylyl cyclase inhibiting pathway, inhibition of adenylate cyclase activity by adrenergic receptor signaling pathway, inhibition of adenylate cyclase activity by adrenergic receptor signalling pathway Relationships: is a type of adenylate cyclase-inhibiting G protein-coupled receptor signaling pathway [GO:0007193]; is a type of GO:0071875 Regulation: regulated by regulation of adenylate cyclase-inhibiting adrenergic receptor signaling pathway [GO:0071877]